negative regulation of dorsal/ventral axon guidance [GO:1905816] (biological process) Relationships: is a type of negative regulation of axon guidance [GO:1902668]; is a type of regulation of dorsal/ventral axon guidance [GO:1905815]; RO_0002212 dorsal/ventral axon guidance [GO:0033563] Also known as: down regulation of dorsal-ventral axon guidance, down regulation of dorsal/ventral axon guidance, down regulation of dorsal/ventral axon pathfinding, down regulation of dorsoventral axon guidance, down-regulation of dorsal-ventral axon guidance, down-regulation of dorsal/ventral axon guidance, down-regulation of dorsal/ventral axon pathfinding, down-regulation of dorsoventral axon guidance, downregulation of dorsal-ventral axon guidance, downregulation of dorsal/ventral axon guidance, downregulation of dorsal/ventral axon pathfinding, downregulation of dorsoventral axon guidance, negative regulation of dorsal-ventral axon guidance, negative regulation of dorsal/ventral axon pathfinding, negative regulation of dorsoventral axon guidance, inhibition of dorsal-ventral axon guidance, inhibition of dorsal/ventral axon guidance, inhibition of dorsal/ventral axon pathfinding, inhibition of dorsoventral axon guidance References: PMID:18434533 Sources: GOC:TermGenie, GO_REF:0000058 Definition: Any process that stops, prevents or reduces the frequency, rate or extent of dorsal/ventral axon guidance.